{
  "term_label": "negative regulation of apoptotic process",
  "gene_symbol": "TSC22D1",
  "gene_name": "TSC22 domain family protein 1",
  "term_id": "GO:0043066",
  "gene": "UniProtKB:Q15714"
}